{
  "gene": "UniProtKB:A0A075B6T6",
  "term_label": "Unknown cellular component",
  "gene_name": "T cell receptor alpha variable 12-2",
  "gene_symbol": "TRAV12-2",
  "term_id": "UNKNOWN:0003"
}